{
  "term_id": "UNKNOWN:0002",
  "gene_symbol": "NARF",
  "gene": "UniProtKB:Q9UHQ1",
  "gene_name": "Nuclear prelamin A recognition factor",
  "term_label": "Unknown biological process"
}